{
  "gene": "UniProtKB:O95424",
  "gene_name": "Dexamethasone-induced protein",
  "term_id": "UNKNOWN:0003",
  "gene_symbol": "DEXI",
  "term_label": "Unknown cellular component"
}